{
  "term_id": "UNKNOWN:0001",
  "gene_name": "Proline-rich protein 20E",
  "term_label": "Unknown molecular function",
  "gene": "UniProtKB:P86478",
  "gene_symbol": "PRR20E"
}